regulation of transformation of host cell by virus [GO:1904187] (biological process) Also known as: regulation of viral transformation, regulation of viral transformation of host cell References: PMID:12200142 Sources: GOC:TermGenie, GO_REF:0000058 Subtypes: negative regulation of transformation of host cell by virus [GO:1904188], positive regulation of transformation of host cell by virus [GO:1904189] Relationships: is a type of regulation of biological process involved in symbiotic interaction [GO:0043903]; regulates symbiont-mediated transformation of host cell [GO:0019087] Definition: Any process that modulates the frequency, rate or extent of transformation of host cell by virus.